{
  "term_label": "DNA damage response",
  "gene": "UniProtKB:P51957",
  "gene_symbol": "NEK4",
  "term_id": "GO:0006974",
  "gene_name": "Serine_threonine-protein kinase Nek4"
}